{
  "gene_name": "Centrosomal protein CEP57L1",
  "gene_symbol": "CEP57L1",
  "gene": "UniProtKB:Q8IYX8",
  "term_label": "Unknown biological process",
  "term_id": "UNKNOWN:0002"
}